{
  "gene_symbol": "EEF1AKMT4-ECE2",
  "gene_name": "EEF1AKMT4-ECE2 readthrough transcript protein",
  "gene": "UniProtKB:P0DPD8",
  "term_id": "GO:0005886",
  "term_label": "plasma membrane"
}